{
  "gene": "UniProtKB:Q8WVD3",
  "term_id": "GO:0061630",
  "gene_name": "E3 ubiquitin-protein ligase RNF138",
  "gene_symbol": "RNF138",
  "term_label": "ubiquitin protein ligase activity"
}